{
  "gene_name": "Lithostathine-1-beta",
  "gene_symbol": "REG1B",
  "term_id": "GO:0005615",
  "gene": "UniProtKB:P48304",
  "term_label": "extracellular space"
}